regulation of leucophore differentiation [GO:0048775] (biological process) Definition: Any process that modulates the frequency, rate or extent of leucophore differentiation. Sources: GOC:mh Relationships: is a type of regulation of pigment cell differentiation [GO:0050932]; regulates leucophore differentiation [GO:0048772] Subtypes: negative regulation of leucophore differentiation [GO:0048776], positive regulation of leucophore differentiation [GO:0048777]